{
  "term_label": "cilium",
  "gene": "UniProtKB:Q9H5P4",
  "gene_symbol": "PDZD7",
  "term_id": "GO:0005929",
  "gene_name": "PDZ domain-containing protein 7"
}